{
  "gene_name": "Extended synaptotagmin-1",
  "term_id": "GO:0008429",
  "gene_symbol": "ESYT1",
  "gene": "UniProtKB:Q9BSJ8",
  "term_label": "phosphatidylethanolamine binding"
}